neuromast mantle cell differentiation [GO:0048888] (biological process) Definition: The process in which a relatively unspecialized cell acquires specialized features of a neuromast mantle cell. Mantle cells are non-sensory cells that surround the sensory strip, separating the neuromast from the epidermis. Mantle cells secrete the cupula in which the ciliary bundles of all of the hair cells are embedded. Relationships: is a type of cell differentiation [GO:0030154]; is part of neuromast development [GO:0048884] Sources: ISBN:0125296509 Subtypes: anterior lateral line neuromast mantle cell differentiation [GO:0048905], GO:0048924